{
  "gene": "UniProtKB:Q76LX8",
  "term_label": "extracellular matrix",
  "gene_symbol": "ADAMTS13",
  "term_id": "GO:0031012",
  "gene_name": "A disintegrin and metalloproteinase with thrombospondin motifs 13"
}